{
  "term_id": "GO:0002486",
  "gene_name": "Retinoic acid early transcript 1E",
  "term_label": "antigen processing and presentation of endogenous peptide antigen via MHC class I via ER pathway, TAP-independent",
  "gene": "UniProtKB:Q8TD07",
  "gene_symbol": "RAET1E"
}